{
  "gene_name": "Peroxisomal targeting signal 2 receptor",
  "term_id": "GO:0005053",
  "gene": "UniProtKB:O00628",
  "gene_symbol": "PEX7",
  "term_label": "peroxisome matrix targeting signal-2 binding"
}